atrioventricular node cell development [GO:0060928] (biological process) Also known as: AV node cell development Sources: GOC:mtg_heart Relationships: is a type of GO:0060926; is part of GO:0060922 Definition: The process whose specific outcome is the progression of an atrioventricular (AV) node cell over time, from its formation to the mature state.